{
  "gene": "UniProtKB:O15440",
  "term_label": "basolateral plasma membrane",
  "gene_symbol": "ABCC5",
  "term_id": "GO:0016323",
  "gene_name": "ATP-binding cassette sub-family C member 5"
}